{
  "gene": "UniProtKB:P53701",
  "term_id": "GO:0005739",
  "gene_name": "Holocytochrome c-type synthase",
  "term_label": "mitochondrion",
  "gene_symbol": "HCCS"
}